{
  "term_label": "tubulin N-terminal-methionine acetyltransferase activity",
  "term_id": "GO:0120519",
  "gene": "UniProtKB:Q9BTE0",
  "gene_symbol": "NAT9",
  "gene_name": "Alpha_beta-tubulin-N-acetyltransferase 9"
}